{
  "term_id": "GO:0005634",
  "term_label": "nucleus",
  "gene_symbol": "PLK5",
  "gene_name": "Inactive serine_threonine-protein kinase PLK5",
  "gene": "UniProtKB:Q496M5"
}